{
  "term_label": "nucleus",
  "gene_symbol": "HSPB8",
  "gene_name": "Heat shock protein beta-8",
  "term_id": "GO:0005634",
  "gene": "UniProtKB:Q9UJY1"
}